{
  "gene": "UniProtKB:P20036",
  "gene_symbol": "HLA-DPA1",
  "term_id": "GO:0042613",
  "gene_name": "HLA class II histocompatibility antigen, DP alpha 1 chain",
  "term_label": "MHC class II protein complex"
}